regulation of platelet-derived growth factor receptor signaling pathway [GO:0010640] (biological process) Relationships: is a type of regulation of signal transduction [GO:0009966]; regulates platelet-derived growth factor receptor signaling pathway [GO:0048008] Sources: GOC:dph, GOC:hjd, GOC:tb Also known as: regulation of platelet-derived growth factor receptor signalling pathway Subtypes: positive regulation of platelet-derived growth factor receptor signaling pathway [GO:0010641], negative regulation of platelet-derived growth factor receptor signaling pathway [GO:0010642], regulation of platelet-derived growth factor receptor-alpha signaling pathway [GO:2000583], regulation of platelet-derived growth factor receptor-beta signaling pathway [GO:2000586] Definition: Any process that modulates the frequency, rate or extent of the platelet-derived growth factor receptor signaling pathway.